{
  "gene_name": "Annexin A4",
  "gene": "UniProtKB:P09525",
  "term_id": "GO:0005544",
  "gene_symbol": "ANXA4",
  "term_label": "calcium-dependent phospholipid binding"
}